Atg1/ULK1 kinase complex [GO:1990316] (cellular component) References: PMID:15743910, PMID:19211835, PMID:19258318, PMID:19597335, PMID:22885598 Sources: GOC:DOS, GOC:bhm, GOC:rb Relationships: is a type of serine/threonine protein kinase complex [GO:1902554]; is part of GO:0005737 Also known as: ATG1 kinase complex, ATG1-ATG13 complex, ATG1/ULK1 signaling complex, Atg1p signalling complex, ULK complex, ULK1 complex, ULK1 signaling complex, ULK1-ATG13-FIP200 complex, ULK1-ATG13-RB1CC1 complex, autophagy-initiation complex Definition: A protein complex consisting of Atg1 (or Atg1 homologs e.g. ULK1, ULK2 in mammals) and Atg13 along with other proteins that regulate its function (e.g. Atg17 in yeast or RB1CC1(FIP200) in mammals). This complex has serine/threonine protein kinase activity and is involved in autophagosome formation.